{
  "gene": "UniProtKB:Q96CM4",
  "term_label": "Unknown molecular function",
  "gene_symbol": "NXNL1",
  "gene_name": "Nucleoredoxin-like protein 1",
  "term_id": "UNKNOWN:0001"
}